negative regulation of retrograde protein transport, ER to cytosol [GO:1904153] (biological process) Definition: Any process that stops, prevents or reduces the frequency, rate or extent of retrograde protein transport, ER to cytosol. References: PMID:18555783 Sources: GOC:PARL, GOC:TermGenie, GOC:bf, GO_REF:0000058 Relationships: is a type of negative regulation of protein exit from endoplasmic reticulum [GO:0070862]; is a type of regulation of retrograde protein transport, ER to cytosol [GO:1904152]; negatively regulates retrograde protein transport, ER to cytosol [GO:0030970] Also known as: down regulation of protein dislocation from ER, down regulation of retrograde protein transport, ER to cytosol, down regulation of retrograde protein transport, endoplasmic reticulum to cytosol, down-regulation of protein dislocation from ER, down-regulation of retrograde protein transport, ER to cytosol, down-regulation of retrograde protein transport, endoplasmic reticulum to cytosol, downregulation of protein dislocation from ER, downregulation of retrograde protein transport, ER to cytosol, downregulation of retrograde protein transport, endoplasmic reticulum to cytosol, negative regulation of protein dislocation from ER, negative regulation of protein retrotranslocation from ER, negative regulation of retrograde protein transport, endoplasmic reticulum to cytosol, inhibition of protein dislocation from ER, inhibition of retrograde protein transport, ER to cytosol, inhibition of retrograde protein transport, endoplasmic reticulum to cytosol